phosphatidylinositol 3-kinase complex, class I [GO:0097651] (cellular component) Subtypes: phosphatidylinositol 3-kinase complex, class IA [GO:0005943], phosphatidylinositol 3-kinase complex, class IB [GO:0005944] References: PMID:24587488 Sources: GOC:ha Definition: A phosphatidylinositol 3-kinase complex that contains a catalytic and a regulatory subunit of a phosphatidylinositol 3-kinase (PI3K) enzyme, plus one or more adaptor proteins. Class I PI3Ks phosphorylate phosphatidylinositol [PI], phosphatidylinositol-4-phosphate [PI(4)P] and phosphatidylinositol-4,5-bisphosphate [PI(4,5)P2], and are divided into subclasses A and B according to the type of adaptor subunit with which they associate. The class I PI3K subfamily of genes comprises members in vertebrates, worm and fly, but none in yeast. Also known as: class I PI3K complex, class I phosphatidylinositol 3-kinase complex Relationships: is a type of phosphatidylinositol 3-kinase complex [GO:0005942]